mitochondrial fission [GO:0000266] (BP) Definition: The division of a mitochondrion within a cell to form two or more separate mitochondrial compartments. Relationships: is a type of mitochondrion organization [GO:0007005]; is a type of organelle fission [GO:0048285] References: PMID:11038192 Also known as: mitochondrial division, mitochondrial proliferation Regulation: regulated by regulation of mitochondrial fission [GO:0090140]; positively regulated by positive regulation of mitochondrial fission [GO:0090141]; negatively regulated by GO:0090258